{
  "gene_name": "Nuclear distribution protein nudE homolog 1",
  "term_id": "GO:0047496",
  "gene_symbol": "NDE1",
  "gene": "UniProtKB:Q9NXR1",
  "term_label": "vesicle transport along microtubule"
}